mesangial cell fate commitment [GO:0072151] (biological process) Subtypes: GO:0072152 Sources: GOC:mtg_kidney_jan10 Relationships: is a type of cell fate commitment [GO:0045165]; is part of mesangial cell differentiation [GO:0072007] Definition: The process in which the developmental fate of a cell becomes restricted such that it will develop into a mesangial cell.